{
  "gene": "UniProtKB:Q9NQ55",
  "term_label": "maturation of LSU-rRNA from tricistronic rRNA transcript (SSU-rRNA, 5.8S rRNA, LSU-rRNA)",
  "term_id": "GO:0000463",
  "gene_symbol": "PPAN",
  "gene_name": "Suppressor of SWI4 1 homolog"
}